{
  "term_id": "UNKNOWN:0002",
  "gene": "UniProtKB:Q93038",
  "term_label": "Unknown biological process",
  "gene_symbol": "TNFRSF25",
  "gene_name": "Tumor necrosis factor receptor superfamily member 25"
}